{
  "term_label": "centrosome",
  "gene": "UniProtKB:H7BZ55",
  "term_id": "GO:0005813",
  "gene_name": "Ciliary rootlet coiled-coil protein 2",
  "gene_symbol": "CROCC2"
}